{
  "gene_symbol": "ALDOC",
  "gene_name": "Fructose-bisphosphate aldolase C",
  "term_id": "GO:0004332",
  "gene": "UniProtKB:P09972",
  "term_label": "fructose-bisphosphate aldolase activity"
}